{
  "term_id": "GO:0007166",
  "term_label": "cell surface receptor signaling pathway",
  "gene_symbol": "TRBV6-9",
  "gene": "UniProtKB:A0A0J9YX75",
  "gene_name": "T cell receptor beta variable 6-9"
}